{
  "gene": "UniProtKB:O95876",
  "gene_name": "WD repeat-containing and planar cell polarity effector protein fritz homolog",
  "term_id": "GO:0007399",
  "term_label": "nervous system development",
  "gene_symbol": "WDPCP"
}